{
  "term_id": "UNKNOWN:0002",
  "gene_symbol": "PSG8",
  "gene_name": "Pregnancy-specific beta-1-glycoprotein 8",
  "term_label": "Unknown biological process",
  "gene": "UniProtKB:Q9UQ74"
}